{
  "term_id": "GO:0008017",
  "gene_symbol": "HOOK2",
  "gene": "UniProtKB:Q96ED9",
  "term_label": "microtubule binding",
  "gene_name": "Protein Hook homolog 2"
}